{
  "gene_name": "Heterogeneous nuclear ribonucleoprotein H3",
  "term_label": "RNA binding",
  "gene": "UniProtKB:P31942",
  "term_id": "GO:0003723",
  "gene_symbol": "HNRNPH3"
}